{
  "term_label": "Unknown cellular component",
  "gene_symbol": "OR9A2",
  "term_id": "UNKNOWN:0003",
  "gene_name": "Olfactory receptor 9A2",
  "gene": "UniProtKB:Q8NGT5"
}